{
  "term_label": "RNA binding",
  "term_id": "GO:0003723",
  "gene_name": "Probable ATP-dependent RNA helicase DHX40",
  "gene": "UniProtKB:Q8IX18",
  "gene_symbol": "DHX40"
}